{
  "term_label": "chloride transmembrane transport",
  "term_id": "GO:1902476",
  "gene_name": "Solute carrier family 12 member 9",
  "gene_symbol": "SLC12A9",
  "gene": "UniProtKB:Q9BXP2"
}